fatty acid alpha-oxidation [GO:0001561] (biological process) References: PMID:10198260 Definition: A metabolic pathway by which 3-methyl branched fatty acids are degraded. These compounds are not degraded by the normal peroxisomal beta-oxidation pathway, because the 3-methyl blocks the dehydrogenation of the hydroxyl group by hydroxyacyl-CoA dehydrogenase. The 3-methyl branched fatty acid is converted in several steps to pristenic acid, which can then feed into the beta-oxidative pathway. Relationships: is a type of GO:0009062; is a type of fatty acid oxidation [GO:0019395]